{
  "gene_symbol": "OR6Y1",
  "gene_name": "Olfactory receptor 6Y1",
  "gene": "UniProtKB:Q8NGX8",
  "term_label": "plasma membrane",
  "term_id": "GO:0005886"
}